{
  "term_id": "GO:0005815",
  "term_label": "microtubule organizing center",
  "gene_symbol": "IFT46",
  "gene": "UniProtKB:Q9NQC8",
  "gene_name": "Intraflagellar transport protein 46 homolog"
}